{
  "term_id": "GO:0001664",
  "gene_symbol": "GNAQ",
  "gene_name": "Guanine nucleotide-binding protein G(q) subunit alpha",
  "gene": "UniProtKB:P50148",
  "term_label": "G protein-coupled receptor binding"
}